FAD metabolic process [GO:0046443] (biological process) References: PMID:20822113 Relationships: is a type of flavin adenine dinucleotide metabolic process [GO:0072387] Definition: The chemical reactions and pathways involving FAD, the oxidized form of flavin adenine dinucleotide. Subtypes: GO:0006747 Also known as: FAD metabolism, oxidized flavin adenine dinucleotide metabolic process, oxidized flavin adenine dinucleotide metabolism, oxidized flavin-adenine dinucleotide metabolic process, oxidized flavin-adenine dinucleotide metabolism